{
  "gene_name": "One cut domain family member 2",
  "gene_symbol": "ONECUT2",
  "term_label": "DNA-binding transcription factor activity, RNA polymerase II-specific",
  "term_id": "GO:0000981",
  "gene": "UniProtKB:O95948"
}